{
  "gene_name": "Roundabout homolog 4",
  "term_label": "axon guidance",
  "gene_symbol": "ROBO4",
  "term_id": "GO:0007411",
  "gene": "UniProtKB:Q8WZ75"
}